pronephric sinus development [GO:0039012] (biological process) References: PMID:10535314 Sources: GOC:mtg_kidney_jan10, XAO:0000385 Definition: The process whose specific outcome is the progression of the pronephric sinus over time, from its formation to the mature structure. The pronephric sinus is an ill-defined capillary network that lies between the pronephric tubules. Relationships: is a type of anatomical structure development [GO:0048856]; is part of pronephros development [GO:0048793]